{
  "term_id": "GO:0007288",
  "gene": "UniProtKB:Q96MT7",
  "gene_name": "Cilia- and flagella-associated protein 44",
  "gene_symbol": "CFAP44",
  "term_label": "sperm axoneme assembly"
}